Cdc42 GTPase complex [GO:0071521] (cellular component) Relationships: is a type of GO:0140535; is a type of GTPase complex [GO:1905360] Definition: A protein complex formed by the association of the small GTPase Cdc42 with additional proteins. In Schizosaccharomyces the complex contains the Cdc42, Ras1, Scd1, Scd2, andShk1 proteins, and functions in the Ras1-Scd GTPase signaling pathway. Also known as: Ras1-Scd1-Scd2-Cdc42-Shk1 complex References: PMID:10567532, PMID:7923372, PMID:8943016 Sources: GOC:mah, GOC:vw